{
  "gene_symbol": "PDK3",
  "term_id": "GO:0005739",
  "term_label": "mitochondrion",
  "gene": "UniProtKB:Q15120",
  "gene_name": "[Pyruvate dehydrogenase (acetyl-transferring)] kinase isozyme 3, mitochondrial"
}